{
  "gene_name": "Histone H3-7",
  "term_id": "GO:0000776",
  "term_label": "kinetochore",
  "gene_symbol": "H3-7",
  "gene": "UniProtKB:Q5TEC6"
}